{
  "term_id": "GO:0006457",
  "gene_name": "Peptidyl-prolyl cis-trans isomerase FKBP9",
  "gene": "UniProtKB:O95302",
  "term_label": "protein folding",
  "gene_symbol": "FKBP9"
}